{
  "gene_symbol": "PHF14",
  "gene": "UniProtKB:O94880",
  "term_label": "Unknown cellular component",
  "term_id": "UNKNOWN:0003",
  "gene_name": "PHD finger protein 14"
}